{
  "gene": "UniProtKB:A6NHS1",
  "gene_name": "Putative uncharacterized protein ENSP00000347057",
  "gene_symbol": "A6NHS1",
  "term_id": "UNKNOWN:0001",
  "term_label": "Unknown molecular function"
}